{
  "gene_name": "Myeloid cell nuclear differentiation antigen",
  "gene": "UniProtKB:P41218",
  "term_label": "nucleolus",
  "gene_symbol": "MNDA",
  "term_id": "GO:0005730"
}